{
  "term_id": "GO:0070059",
  "gene": "UniProtKB:Q9H0C3",
  "gene_symbol": "TMEM117",
  "gene_name": "Transmembrane protein 117",
  "term_label": "intrinsic apoptotic signaling pathway in response to endoplasmic reticulum stress"
}